{
  "gene": "UniProtKB:Q8N2Y8",
  "term_label": "cytoplasmic vesicle",
  "gene_name": "AP-4 complex accessory subunit RUSC2",
  "gene_symbol": "RUSC2",
  "term_id": "GO:0031410"
}